polar microtubule [GO:0005827] (cellular component) Sources: ISBN:0815316194 Also known as: pole-to-pole microtubule Definition: Any of the spindle microtubules that come from each pole and overlap at the spindle midzone. This interdigitating structure consisting of antiparallel microtubules is responsible for pushing the poles of the spindle apart. Relationships: is a type of spindle microtubule [GO:0005876]; is part of spindle pole [GO:0000922] Subtypes: GO:1990537